histone H1-4S27 kinase activity [GO:0140197] (MF) Definition: Catalysis of the reaction: histone H1-4-serine (position 187) + ATP = histone H1-4-phosphoserine (position 187) + ADP. Relationships: is a type of protein serine/threonine kinase activity [GO:0004674]; is a type of histone H1 kinase activity [GO:0140190] References: PMID:21511733, PMID:21852232, PMID:33238524